{
  "term_id": "GO:0047238",
  "gene_name": "Chondroitin sulfate synthase 3",
  "gene": "UniProtKB:Q70JA7",
  "term_label": "glucuronosyl-N-acetylgalactosaminyl-proteoglycan 4-beta-N-acetylgalactosaminyltransferase activity",
  "gene_symbol": "CHSY3"
}